{
  "gene_name": "Transcription factor p65",
  "term_id": "GO:0045087",
  "gene": "UniProtKB:Q04206",
  "gene_symbol": "RELA",
  "term_label": "innate immune response"
}